{
  "gene_symbol": "TSTD2",
  "term_id": "UNKNOWN:0002",
  "gene_name": "Thiosulfate sulfurtransferase_rhodanese-like domain-containing protein 2",
  "term_label": "Unknown biological process",
  "gene": "UniProtKB:Q5T7W7"
}